{
  "term_label": "lymph vessel morphogenesis",
  "gene": "UniProtKB:Q4LDE5",
  "gene_symbol": "SVEP1",
  "gene_name": "Sushi, von Willebrand factor type A, EGF and pentraxin domain-containing protein 1",
  "term_id": "GO:0036303"
}